iron-sulfur cluster transfer complex [GO:1990230] (cellular component) Also known as: Fe-S cluster transfer complex, IscA complex, SufA complex, SufA dimer Definition: A protein complex capable of catalyzing the transfer of an iron-sulfur (Fe-S) cluster from one compound (donor) to another (acceptor), which may be a target protein or another Fe-S assembly complex. In humans, it consists of HSPA9, HSCB, GLRX5, ABCB7 and GFER. Relationships: is a type of transferase complex [GO:1990234] References: PMID:19810706, PMID:34660592 Sources: GOC:bhm